{
  "term_label": "mRNA cis splicing, via spliceosome",
  "gene": "UniProtKB:O95391",
  "term_id": "GO:0045292",
  "gene_name": "Pre-mRNA-splicing factor SLU7",
  "gene_symbol": "SLU7"
}